{
  "gene_symbol": "CD44",
  "gene": "UniProtKB:P16070",
  "term_label": "macrophage migration inhibitory factor receptor complex",
  "gene_name": "CD44 antigen",
  "term_id": "GO:0035692"
}